{
  "gene": "UniProtKB:P47870",
  "gene_name": "Gamma-aminobutyric acid receptor subunit beta-2",
  "term_id": "GO:1902476",
  "gene_symbol": "GABRB2",
  "term_label": "chloride transmembrane transport"
}